endopeptidase regulator activity [GO:0061135] (molecular function) Sources: GOC:dph, GOC:tb Relationships: is a type of peptidase regulator activity [GO:0061134]; RO_0002211 endopeptidase activity [GO:0004175] Definition: Binds to and modulates the activity of a peptidase, any enzyme that hydrolyzes nonterminal peptide bonds in polypeptides. Subtypes: endopeptidase inhibitor activity [GO:0004866], endopeptidase activator activity [GO:0061133]